{
  "term_label": "transcription cis-regulatory region binding",
  "gene": "UniProtKB:Q6ZN55",
  "term_id": "GO:0000976",
  "gene_symbol": "ZNF574",
  "gene_name": "Zinc finger protein 574"
}